centrosome duplication [GO:0051298] (biological process) Relationships: is a type of GO:0022402; is part of GO:0007098 Also known as: centrosome replication Regulation: regulated by regulation of centrosome duplication [GO:0010824]; positively regulated by positive regulation of centrosome duplication [GO:0010825]; negatively regulated by negative regulation of centrosome duplication [GO:0010826] Sources: GOC:ai Definition: The replication of a centrosome, a structure comprised of a pair of centrioles and peri-centriolar material from which a microtubule spindle apparatus is organized.